{
  "term_id": "GO:0042981",
  "gene": "UniProtKB:Q8N1N2",
  "term_label": "regulation of apoptotic process",
  "gene_name": "Dynactin-associated protein",
  "gene_symbol": "DYNAP"
}